L-alanine transmembrane transporter activity [GO:0015180] (molecular function) Relationships: is a type of L-amino acid transmembrane transporter activity [GO:0015179]; is a type of GO:0022858; BFO_0000050 GO:0015808 Also known as: L-alanine transporter activity Subtypes: L-alanine:proton antiporter activity [GO:0140407] Definition: Enables the transfer of L-alanine from one side of a membrane to the other. L-alanine is the L-enantiomer of 2-aminopropanoic acid. Sources: GOC:go_curators, GOC:jsg, GOC:mah, GOC:mtg_transport, ISBN:0198506732